{
  "gene_name": "Cell division cycle-associated protein 3",
  "term_label": "Unknown molecular function",
  "gene": "UniProtKB:Q99618",
  "term_id": "UNKNOWN:0001",
  "gene_symbol": "CDCA3"
}